antennal development [GO:0007469] (biological process) Definition: The process whose specific outcome is the progression of the antenna over time, from its formation to the mature structure. The antenna are the sensory structures on the head that are capable of detecting various environmental stimuli. Sources: http://fly.ebi.ac.uk/.bin/cvreport2?id=FBcv0004526 Relationships: is a type of GO:0035114; is part of eye-antennal disc development [GO:0035214]